{
  "term_label": "apical plasma membrane",
  "gene_symbol": "NHERF1",
  "gene": "UniProtKB:O14745",
  "gene_name": "Na(+)_H(+) exchange regulatory cofactor NHE-RF1",
  "term_id": "GO:0016324"
}